{
  "gene_symbol": "VSIG8",
  "gene_name": "V-set and immunoglobulin domain-containing protein 8",
  "term_id": "UNKNOWN:0002",
  "term_label": "Unknown biological process",
  "gene": "UniProtKB:P0DPA2"
}